{
  "gene": "UniProtKB:P36888",
  "term_id": "GO:0043235",
  "gene_symbol": "FLT3",
  "term_label": "receptor complex",
  "gene_name": "Receptor-type tyrosine-protein kinase FLT3"
}